oxidoreductase activity, acting on paired donors, with incorporation or reduction of molecular oxygen, NAD(P)H as one donor, and incorporation of two atoms of oxygen into one donor [GO:0016708] (molecular function) Relationships: is a type of GO:0016705; is a type of GO:0051213 Sources: EC:1.14.12.- Definition: Catalysis of an oxidation-reduction (redox) reaction in which hydrogen or electrons are transferred from NADH or NADPH and one other donor, and two atoms of oxygen are incorporated into one donor. Subtypes: 3-phenylpropionate dioxygenase activity [GO:0008695], nitric oxide dioxygenase NAD(P)H activity [GO:0008941], carbazole 1,9a-dioxygenase [NAD(P)H] activity [GO:0018564], dibenzofuran 4,4a-dioxygenase activity [GO:0018610], trihydroxytoluene dioxygenase activity [GO:0018616], anthranilate 1,2-dioxygenase (deaminating, decarboxylating) activity [GO:0018618], benzene 1,2-dioxygenase activity [GO:0018619], GO:0018620, 4-sulfobenzoate 3,4-dioxygenase activity [GO:0018621], GO:0018622, benzoate 1,2-dioxygenase activity [GO:0018623], GO:0018624, naphthalene 1,2-dioxygenase activity [GO:0018625], 2-halobenzoate 1,2-dioxygenase activity [GO:0018626], 2-aminobenzenesulfonate 2,3-dioxygenase activity [GO:0018627], GO:0018628, 2-hydroxyquinoline 5,6-dioxygenase activity [GO:0018629], GO:0018687, 3-hydroxy-2-methylpyridinecarboxylate dioxygenase activity [GO:0047081], 3-chlorobenzoate-4,5-oxygenase activity [GO:0102044], 3-chlorobenzoate-3,4-oxygenase activity [GO:0102045], 3,4-dichlorobenzoate-4,5-oxygenase activity [GO:0102046] Also known as: oxidoreductase activity, acting on paired donors, with incorporation or reduction of molecular oxygen, NADH or NADPH as one donor, and incorporation of two atoms of oxygen into one donor